{
  "term_label": "voltage-gated calcium channel activity",
  "term_id": "GO:0005245",
  "gene": "UniProtKB:Q5VU97",
  "gene_symbol": "CACHD1",
  "gene_name": "VWFA and cache domain-containing protein 1"
}